{
  "term_id": "UNKNOWN:0001",
  "gene_name": "Shugoshin 2",
  "gene_symbol": "SGO2",
  "term_label": "Unknown molecular function",
  "gene": "UniProtKB:Q562F6"
}